negative regulation of embryonic pattern specification [GO:1902876] (biological process) Definition: Any process that stops, prevents or reduces the frequency, rate or extent of embryonic pattern specification. Also known as: down regulation of embryonic pattern specification, down-regulation of embryonic pattern specification, downregulation of embryonic pattern specification, inhibition of embryonic pattern specification, down regulation of ventral/lateral system, down-regulation of ventral/lateral system, downregulation of ventral/lateral system, inhibition of ventral/lateral system, negative regulation of ventral/lateral system Relationships: is_a negative regulation of multicellular organismal process [GO:0051241]; is_a regulation of embryonic pattern specification [GO:1902875]; RO_0002212 GO:0009880 References: PMID:16872597 Sources: GOC:TermGenie, GOC:mr, GO_REF:0000058